{
  "gene_symbol": "FIBCD1",
  "term_label": "Unknown biological process",
  "gene": "UniProtKB:Q8N539",
  "gene_name": "Fibrinogen C domain-containing protein 1",
  "term_id": "UNKNOWN:0002"
}